RHG protein domain binding [GO:0089719] (molecular function) Sources: GOC:dos, GOC:ha Also known as: RHG domain binding, iap binding domain binding, inhibitor of apoptosis binding domain binding, reaper hid grim domain binding Definition: Binding to an RHG (reaper/hid/grimm) domain/motif (AKA iap binding motif). Relationships: is a type of protein binding [GO:0005515]